{
  "gene_name": "Baculoviral IAP repeat-containing protein 2",
  "term_label": "cytoplasm",
  "term_id": "GO:0005737",
  "gene_symbol": "BIRC2",
  "gene": "UniProtKB:Q13490"
}